{
  "gene": "UniProtKB:Q92922",
  "gene_symbol": "SMARCC1",
  "term_label": "SWI/SNF complex",
  "term_id": "GO:0016514",
  "gene_name": "SWI_SNF complex subunit SMARCC1"
}